cleavage between 2S rRNA and LSU-rRNA of tetracistronic rRNA transcript (SSU-rRNA, 5.8S rRNA, 2S rRNA, LSU-rRNA) [GO:0000485] (biological process) References: PMID:768488 Sources: GOC:curators Definition: Endonucleolytic cleavage between the LSU-rRNA and the 2S rRNA of an rRNA molecule originally produced as a tetracistronic rRNA transcript that contained the Small SubUnit (SSU) rRNA, the 5.8S rRNA, 2S rRNA, and the Large SubUnit (LSU) rRNA, in that order, from 5' to 3' along the primary transcript. Relationships: is a type of endonucleolytic cleavage of tetracistronic rRNA transcript (SSU-rRNA, 5.8S rRNA, 2S rRNA, LSU-rRNA) [GO:0000483]; is part of maturation of LSU-rRNA from tetracistronic rRNA transcript (SSU-rRNA, 5.8S rRNA, 2S rRNA, LSU-rRNA) [GO:0000473]; is part of maturation of 2S rRNA [GO:0000475]